indole-containing compound biosynthetic process [GO:0042435] (biological process) Definition: The chemical reactions and pathways resulting in the formation of compounds that contain an indole (2,3-benzopyrrole) skeleton. Subtypes: indoleacetic acid biosynthetic process [GO:0009684], indole phytoalexin biosynthetic process [GO:0009700], indole glucosinolate biosynthetic process [GO:0009759], melatonin biosynthetic process [GO:0030187], GO:0033474, serotonin biosynthetic process [GO:0042427], GO:0042432, indolalkylamine biosynthetic process [GO:0046219], psilocybin biosynthetic process [GO:0140380], tryprostatin A biosynthetic process [GO:0140654], brevianamide F biosynthetic process [GO:1900805] Also known as: indole derivative biosynthesis, indole derivative biosynthetic process, indole-containing compound anabolism, indole-containing compound biosynthesis, indole-containing compound formation, indole-containing compound synthesis Sources: GOC:jl Relationships: is a type of biosynthetic process [GO:0009058]; is_a indole-containing compound metabolic process [GO:0042430]